{
  "gene_name": "Pre-B-cell leukemia transcription factor 1",
  "term_id": "GO:0048568",
  "gene_symbol": "PBX1",
  "term_label": "embryonic organ development",
  "gene": "UniProtKB:P40424"
}